{
  "term_id": "GO:0006357",
  "term_label": "regulation of transcription by RNA polymerase II",
  "gene_symbol": "ZNF316",
  "gene_name": "Zinc finger protein 316",
  "gene": "UniProtKB:A6NFI3"
}